metabolite repair [GO:0110051] (biological process) Subtypes: toxic metabolite repair [GO:0110052] Relationships: is a type of GO:0008152 References: PMID:23334546, PMID:28373563 Sources: GOC:ka Definition: A cellular process that, through single- or multi-step enzymatic reactions, repairs useless or toxic endogenous compounds, formed as by-products of primary metabolism, by converting them into useful metabolites.